{
  "gene": "UniProtKB:Q9Y6U7",
  "gene_symbol": "RNF215",
  "term_label": "cytoplasm",
  "term_id": "GO:0005737",
  "gene_name": "RING finger protein 215"
}